{
  "term_id": "GO:0005634",
  "term_label": "nucleus",
  "gene_name": "Transcription factor GATA-6",
  "gene_symbol": "GATA6",
  "gene": "UniProtKB:Q92908"
}